{
  "term_id": "GO:0045893",
  "gene_symbol": "MLLT11",
  "gene_name": "Protein AF1q",
  "term_label": "positive regulation of DNA-templated transcription",
  "gene": "UniProtKB:Q13015"
}